positive regulation of neuroblast proliferation [GO:0002052] (biological process) Relationships: is a type of positive regulation of neurogenesis [GO:0050769]; is a type of regulation of neuroblast proliferation [GO:1902692]; is a type of GO:2000179; positively regulates neuroblast proliferation [GO:0007405] Definition: Any process that activates or increases the rate of neuroblast proliferation. Sources: GOC:dph Also known as: up regulation of neuroblast proliferation, up-regulation of neuroblast proliferation, upregulation of neuroblast proliferation, activation of neuroblast proliferation, stimulation of neuroblast proliferation